aerobic phenol-containing compound catabolic process [GO:0046191] (biological process) Definition: The chemical reactions and pathways resulting in the breakdown of a phenol, any compound containing one or more hydroxyl groups directly attached to an aromatic carbon ring, in the presence of oxygen. Also known as: aerobic phenol-containing compound breakdown, aerobic phenol-containing compound catabolism, aerobic phenol-containing compound degradation Relationships: is_a phenol-containing compound catabolic process [GO:0019336] Sources: GOC:ai